{
  "term_id": "GO:0009052",
  "gene": "UniProtKB:Q96AT9",
  "gene_name": "Ribulose-phosphate 3-epimerase",
  "gene_symbol": "RPE",
  "term_label": "pentose-phosphate shunt, non-oxidative branch"
}